{
  "term_id": "GO:0004867",
  "gene_symbol": "SERPINB2",
  "gene_name": "Plasminogen activator inhibitor 2",
  "gene": "UniProtKB:P05120",
  "term_label": "serine-type endopeptidase inhibitor activity"
}